{
  "gene_symbol": "FAM13A",
  "term_id": "UNKNOWN:0002",
  "gene": "UniProtKB:O94988",
  "term_label": "Unknown biological process",
  "gene_name": "Protein FAM13A"
}